{
  "term_id": "GO:0000785",
  "term_label": "chromatin",
  "gene_symbol": "EOMES",
  "gene": "UniProtKB:O95936",
  "gene_name": "Eomesodermin homolog"
}